negative regulation of systemic arterial blood pressure [GO:0003085] (biological process) Sources: GOC:mtg_cardio Definition: The process that reduces the force with which blood travels through the systemic arterial circulatory system. Subtypes: baroreceptor response to increased systemic arterial blood pressure [GO:0001983], norepinephrine-epinephrine-mediated vasodilation involved in regulation of systemic arterial blood pressure [GO:0002025], GO:0002033, regulation of systemic arterial blood pressure by stress relaxation [GO:0003046], acetylcholine-mediated vasodilation involved in regulation of systemic arterial blood pressure [GO:0003069] Relationships: is_a negative regulation of blood pressure [GO:0045776]; is part of GO:0003073